regulation of necroptotic process [GO:0060544] (biological process) Definition: Any process that modulates the rate, frequency or extent of a necroptotic process, a necrotic cell death process that results from the activation of endogenous cellular processes, such as signaling involving death domain receptors or Toll-like receptors. Sources: GOC:BHF, GOC:dph, GOC:mtg_apoptosis, GOC:tb Also known as: regulation of necroptosis Relationships: is a type of GO:0062098; regulates necroptotic process [GO:0070266] Subtypes: positive regulation of necroptotic process [GO:0060545], negative regulation of necroptotic process [GO:0060546]